{
  "gene_name": "Lysine-rich coiled-coil protein 1",
  "gene_symbol": "KRCC1",
  "term_id": "UNKNOWN:0001",
  "gene": "UniProtKB:Q9NPI7",
  "term_label": "Unknown molecular function"
}